4-methyleneglutaminase activity [GO:0047582] (molecular function) Definition: Catalysis of the reaction: 4-methylene-L-glutamine + H2O = 4-methylene-L-glutamate + NH4. Relationships: is a type of hydrolase activity, acting on carbon-nitrogen (but not peptide) bonds, in linear amides [GO:0016811] Also known as: 4-methylene-L-glutamine amidohydrolase activity, 4-methyleneglutamine amidohydrolase activity, 4-methyleneglutamine deamidase activity Sources: EC:3.5.1.67, RHEA:14741